{
  "gene_symbol": "TARBP2",
  "gene_name": "RISC-loading complex subunit TARBP2",
  "term_id": "GO:0035197",
  "term_label": "siRNA binding",
  "gene": "UniProtKB:Q15633"
}